{
  "gene_symbol": "RADIL",
  "term_id": "GO:0051020",
  "gene_name": "Ras-associating and dilute domain-containing protein",
  "gene": "UniProtKB:Q96JH8",
  "term_label": "GTPase binding"
}